{
  "term_label": "digestive tract development",
  "gene_name": "Nipped-B-like protein",
  "term_id": "GO:0048565",
  "gene": "UniProtKB:Q6KC79",
  "gene_symbol": "NIPBL"
}